{
  "gene_symbol": "SMAD2",
  "gene_name": "Mothers against decapentaplegic homolog 2",
  "term_label": "transforming growth factor beta receptor signaling pathway",
  "gene": "UniProtKB:Q15796",
  "term_id": "GO:0007179"
}